{
  "term_id": "UNKNOWN:0001",
  "term_label": "Unknown molecular function",
  "gene_name": "Putative ATP-dependent RNA helicase TDRD12",
  "gene": "UniProtKB:Q587J7",
  "gene_symbol": "TDRD12"
}